{
  "gene_symbol": "VOPP1",
  "gene_name": "Vesicular, overexpressed in cancer, prosurvival protein 1",
  "gene": "UniProtKB:Q96AW1",
  "term_id": "UNKNOWN:0002",
  "term_label": "Unknown biological process"
}